{
  "gene_name": "E3 ubiquitin-protein ligase TRIM32",
  "gene": "UniProtKB:Q13049",
  "gene_symbol": "TRIM32",
  "term_label": "positive regulation of tumor necrosis factor-mediated signaling pathway",
  "term_id": "GO:1903265"
}